notochord morphogenesis [GO:0048570] (BP) Sources: GOC:jid Definition: The process in which the anatomical structures of the notochord are generated and organized. The notochord is a mesoderm-derived structure located ventral of the developing nerve cord. In vertebrates, the notochord serves as a core around which other mesodermal cells form the vertebrae. In the most primitive chordates, which lack vertebrae, the notochord persists as a substitute for a vertebral column. Relationships: is_a embryonic organ morphogenesis [GO:0048562]; BFO_0000050 notochord development [GO:0030903]